{
  "gene_name": "Histidine decarboxylase",
  "term_id": "GO:0001694",
  "term_label": "histamine biosynthetic process",
  "gene": "UniProtKB:P19113",
  "gene_symbol": "HDC"
}